dopamine uptake [GO:0090494] (biological process) Definition: The directed movement of dopamine into a cell. Relationships: is a type of GO:0015872; is a type of catecholamine uptake [GO:0090493] Subtypes: dopamine uptake involved in synaptic transmission [GO:0051583] Sources: GOC:dph, GOC:tb